endoplasmic reticulum Sec complex [GO:0031205] (CC) Relationships: is a type of GO:0098796; is a type of endoplasmic reticulum protein-containing complex [GO:0140534]; is part of rough endoplasmic reticulum membrane [GO:0030867]; has part Sec61 translocon complex [GO:0005784] Definition: An endoplasmic reticulum membrane-associated complex involved in the translocation of proteins that are targeted to the ER. In yeast, this complex consists of two subcomplexes, namely, the Sec61 complex and the Sec62/Sec63 complex. References: PMID:14617809 Sources: GOC:mtg_sensu